{
  "gene_symbol": "SNX9",
  "term_label": "cleavage furrow formation",
  "gene": "UniProtKB:Q9Y5X1",
  "term_id": "GO:0036089",
  "gene_name": "Sorting nexin-9"
}